{
  "gene": "UniProtKB:Q96K78",
  "term_id": "GO:0004930",
  "gene_symbol": "ADGRG7",
  "gene_name": "Adhesion G-protein coupled receptor G7",
  "term_label": "G protein-coupled receptor activity"
}